{
  "gene": "UniProtKB:Q13191",
  "term_id": "GO:0061630",
  "term_label": "ubiquitin protein ligase activity",
  "gene_symbol": "CBLB",
  "gene_name": "E3 ubiquitin-protein ligase CBL-B"
}